{
  "term_id": "GO:0031507",
  "term_label": "heterochromatin formation",
  "gene_symbol": "SMARCA1",
  "gene_name": "Probable global transcription activator SNF2L1",
  "gene": "UniProtKB:P28370"
}